regulation of protein catabolic process at synapse, modulating synaptic transmission [GO:0099574] (biological process) Relationships: is a type of modulation of chemical synaptic transmission [GO:0050804]; is a type of regulation protein catabolic process at synapse [GO:0140250] Note: Note that this term was created for the SynGO project, and will be obsoleted when the SynGO annotations are made in Noctua. Definition: Any process that modulates synaptic transmission by regulating protein degradation at the synapse. Sources: GOC:dos